{
  "gene": "UniProtKB:Q9Y484",
  "gene_name": "WD repeat domain phosphoinositide-interacting protein 4",
  "gene_symbol": "WDR45",
  "term_label": "glycophagy",
  "term_id": "GO:0061723"
}